{
  "gene_name": "NADH-ubiquinone oxidoreductase chain 2",
  "gene": "UniProtKB:P03891",
  "term_label": "respiratory chain complex I",
  "term_id": "GO:0045271",
  "gene_symbol": "MT-ND2"
}